singlet oxygen-mediated programmed cell death [GO:0010343] (biological process) Relationships: is a type of programmed cell death in response to reactive oxygen species [GO:0097468]; is part of cellular response to singlet oxygen [GO:0071452] References: PMID:17075038 Sources: GOC:mtg_apoptosis Also known as: light-dependent programmed cell death, programmed cell death in response to singlet oxygen Definition: Programmed cell death induced by singlet oxygen. Programmed cell death is the cell death resulting from activation of endogenous cellular processes.